{
  "gene_name": "Zinc finger protein 107",
  "gene_symbol": "ZNF107",
  "term_label": "nucleus",
  "term_id": "GO:0005634",
  "gene": "UniProtKB:Q9UII5"
}